{
  "term_label": "detection of stimulus",
  "term_id": "GO:0051606",
  "gene": "UniProtKB:Q9BY67",
  "gene_symbol": "CADM1",
  "gene_name": "Cell adhesion molecule 1"
}